{
  "term_id": "GO:0033130",
  "gene_symbol": "LY6H",
  "term_label": "acetylcholine receptor binding",
  "gene_name": "Lymphocyte antigen 6H",
  "gene": "UniProtKB:O94772"
}